mammary gland specification [GO:0060594] (biological process) Also known as: mammary line specification Definition: The regionalization process in which the mammary line is specified. The mammary line is a ridge of epidermal cells that will form the mammary placodes. Relationships: is a type of specification of animal organ identity [GO:0010092]; is_a mammary gland formation [GO:0060592] Sources: GOC:dph